{
  "term_id": "UNKNOWN:0002",
  "gene_symbol": "C1QTNF6",
  "gene_name": "Complement C1q tumor necrosis factor-related protein 6",
  "term_label": "Unknown biological process",
  "gene": "UniProtKB:Q9BXI9"
}